{
  "gene_name": "Vacuolar protein sorting-associated protein 37D",
  "gene_symbol": "VPS37D",
  "term_id": "GO:0043162",
  "term_label": "ubiquitin-dependent protein catabolic process via the multivesicular body sorting pathway",
  "gene": "UniProtKB:Q86XT2"
}